{
  "gene_name": "Zinc finger protein 835",
  "term_label": "DNA-binding transcription factor activity",
  "gene_symbol": "ZNF835",
  "term_id": "GO:0003700",
  "gene": "UniProtKB:Q9Y2P0"
}